{
  "gene": "UniProtKB:Q8TE76",
  "term_id": "GO:0140002",
  "gene_name": "MORC family CW-type zinc finger protein 4",
  "term_label": "histone H3K4me3 reader activity",
  "gene_symbol": "MORC4"
}